{
  "gene_symbol": "OR8U3",
  "gene": "UniProtKB:Q8NH85",
  "gene_name": "Olfactory receptor 8U3",
  "term_label": "Unknown molecular function",
  "term_id": "UNKNOWN:0001"
}